{
  "gene_name": "Mitogen-activated protein kinase 12",
  "gene": "UniProtKB:P53778",
  "term_id": "GO:0004674",
  "gene_symbol": "MAPK12",
  "term_label": "protein serine/threonine kinase activity"
}